{
  "gene_name": "Regulatory factor X-associated protein",
  "gene": "UniProtKB:O00287",
  "term_id": "GO:0005634",
  "term_label": "nucleus",
  "gene_symbol": "RFXAP"
}